{
  "term_label": "cytoplasm",
  "gene_name": "Fidgetin",
  "gene_symbol": "FIGN",
  "term_id": "GO:0005737",
  "gene": "UniProtKB:Q5HY92"
}